{
  "gene_symbol": "PTPRO",
  "term_label": "glutamatergic synapse",
  "term_id": "GO:0098978",
  "gene": "UniProtKB:Q16827",
  "gene_name": "Receptor-type tyrosine-protein phosphatase O"
}